{
  "gene_name": "Protein-L-histidine N-pros-methyltransferase",
  "gene_symbol": "METTL9",
  "term_label": "protein-L-histidine N-pros-methyltransferase activity",
  "gene": "UniProtKB:Q9H1A3",
  "term_id": "GO:0106370"
}